ciliary pocket collar [GO:1990900] (cellular component) Note: Note that a 'flagellar collar' is described in Choanoflagellates, but this is different from the ciliary pocket collar found e.g. in Giardia; in Choanoflagellates, a single apical flagellum is surrounded by a collar of 30-40 microvilli. References: PMID:18462016, PMID:19806154 Sources: GOC:giardia Definition: A constriction site at the junction of the plasma, flagellar and flagellar pocket membranes where the flagellum emerges from the cell body. Observed in some unicellular eukaryotic species such as Chlamydomonas, Giardia and Trypanosoma. Relationships: is a type of cellular anatomical structure [GO:0110165]; BFO_0000050 ciliary pocket [GO:0020016] Also known as: cilium pocket collar, flagellar pocket collar, flagellum pocket collar, FPC, flagellar collar, flagellar pore